{
  "term_id": "GO:0005654",
  "gene_name": "Rho GTPase-activating protein 4",
  "gene": "UniProtKB:P98171",
  "gene_symbol": "ARHGAP4",
  "term_label": "nucleoplasm"
}